{
  "gene_symbol": "IGHV1-18",
  "gene_name": "Immunoglobulin heavy variable 1-18",
  "gene": "UniProtKB:A0A0C4DH31",
  "term_id": "GO:0016064",
  "term_label": "immunoglobulin mediated immune response"
}